{
  "term_label": "hormone activity",
  "gene": "UniProtKB:Q06141",
  "gene_name": "Regenerating islet-derived protein 3-alpha",
  "gene_symbol": "REG3A",
  "term_id": "GO:0005179"
}